{
  "term_label": "Unknown biological process",
  "gene_symbol": "GARIN4",
  "gene": "UniProtKB:Q8IYT1",
  "gene_name": "Golgi-associated RAB2 interactor protein 4",
  "term_id": "UNKNOWN:0002"
}